negative regulation of immunological synapse formation [GO:2000521] (biological process) Relationships: is a type of negative regulation of lymphocyte activation [GO:0051250]; is a type of regulation of immunological synapse formation [GO:2000520]; RO_0002212 immunological synapse formation [GO:0001771] Also known as: negative regulation of formation of immunological synapse Sources: GOC:obol Definition: Any process that stops, prevents or reduces the frequency, rate or extent of immunological synapse formation.